{
  "gene_symbol": "PLA2G2A",
  "term_id": "GO:0046470",
  "term_label": "phosphatidylcholine metabolic process",
  "gene_name": "Phospholipase A2, membrane associated",
  "gene": "UniProtKB:P14555"
}